regulation of cardioblast cell fate specification [GO:0042686] (biological process) Subtypes: negative regulation of cardioblast cell fate specification [GO:0009997] Sources: GOC:go_curators Definition: Any process that mediates the specification of a cell into a cardioblast. A cardioblast is a cardiac precursor cell. It is a cell that has been committed to a cardiac fate, but will undergo more cell division rather than terminally differentiating. Relationships: is a type of regulation of cardioblast differentiation [GO:0051890]; is a type of regulation of cardiac cell fate specification [GO:2000043]; regulates cardioblast cell fate specification [GO:0042685]